(R)-mandelate catabolic process to catechol [GO:0019598] (biological process) Definition: The chemical reactions and pathways resulting in the breakdown of (R)-mandelate into other compounds, including catechol. Also known as: (R)-mandelate breakdown to catechol, (R)-mandelate degradation to catechol Relationships: is_a catechol-containing compound biosynthetic process [GO:0009713]; is a type of mandelate catabolic process [GO:0019596] Sources: GOC:go_curators